actin filament severing [GO:0051014] (biological process) Also known as: F-actin severing, actin filament severing activity, barbed-end actin capping/severing activity Subtypes: actin filament debranching [GO:0071846] References: PMID:14657234 Sources: GOC:ai Regulation: regulated by regulation of actin filament severing [GO:1903918]; negatively regulated by GO:1903919; positively regulated by positive regulation of actin filament severing [GO:1903920] Relationships: is a type of actin filament-based process [GO:0030029] Definition: The process in which an actin filament is broken down into smaller filaments.